deisopropylhydroxyatrazine aminohydrolase activity [GO:0018757] (molecular function) Definition: Catalysis of the reaction: deisopropylhydroxyatrazine + H2O = NH3 + 2,4-dihydroxy-6-(N'-ethyl)amino-1,3,5-triazine. Sources: UM-BBD_reactionID:r0121 Relationships: is_a hydrolase activity, acting on carbon-nitrogen (but not peptide) bonds, in linear amidines [GO:0016813]